CD40 signaling pathway [GO:0023035] (biological process) References: PMID:11348017 Sources: GOC:mtg_signal, GOC:signaling Regulation: regulated by regulation of CD40 signaling pathway [GO:2000348]; negatively regulated by GO:2000349; positively regulated by positive regulation of CD40 signaling pathway [GO:2000350] Also known as: CD40 signalling pathway Relationships: is a type of GO:0007166 Definition: The series of molecular signals initiated by the binding of the cell surface receptor CD40 to one of its physiological ligands, and ending with the regulation of a downstream cellular process, e.g. transcription.